macronucleus [GO:0031039] (cellular component) Relationships: is a type of nucleus [GO:0005634] Sources: GOC:ns Definition: A membrane-bounded organelle of ciliated protozoan cells that contains polyploid copies of a portion of the cell's complete genome. Transcription of genes occurs in macronuclei. Some ciliate species may contain multiple macronuclei per cell.